plasma membrane proton-transporting ATP synthase complex assembly [GO:0033616] (biological process) Definition: The aggregation, arrangement and bonding together of a proton-transporting ATP synthase in the plasma membrane. Relationships: is a type of proton-transporting ATP synthase complex assembly [GO:0043461]; is part of plasma membrane organization [GO:0007009]; BFO_0000066 plasma membrane [GO:0005886] Sources: GOC:mah